{
  "term_id": "GO:0043066",
  "gene": "UniProtKB:Q8TEJ3",
  "term_label": "negative regulation of apoptotic process",
  "gene_name": "E3 ubiquitin-protein ligase SH3RF3",
  "gene_symbol": "SH3RF3"
}